{
  "gene_symbol": "TERF2",
  "term_label": "telomerase activity",
  "gene": "UniProtKB:Q15554",
  "gene_name": "Telomeric repeat-binding factor 2",
  "term_id": "GO:0003720"
}